negative regulation of anti-Mullerian hormone signaling pathway [GO:1902613] (biological process) References: PMID:23624077 Sources: GOC:TermGenie, GOC:hjd, GO_REF:0000058 Also known as: down regulation of anti-Mullerian hormone signaling pathway, down-regulation of anti-Mullerian hormone signaling pathway, downregulation of anti-Mullerian hormone signaling pathway, inhibition of anti-Mullerian hormone signaling pathway Relationships: is a type of GO:0090101; is a type of regulation of anti-Mullerian hormone signaling pathway [GO:1902612]; negatively regulates anti-Mullerian hormone receptor signaling pathway [GO:1990262] Definition: Any process that stops, prevents or reduces the frequency, rate or extent of anti-Mullerian hormone signaling pathway.